mitochondrial RNA localization [GO:0019093] (biological process) Relationships: is_a RNA localization [GO:0006403]; occurs in mitochondrion [GO:0005739] Definition: Any process in which mitochondrial RNA is transported to, or maintained in, a specific location. Sources: GOC:ai Subtypes: pole plasm mitochondrial rRNA localization [GO:0019095] Also known as: establishment and maintenance of mitochondrial RNA localization, mitochondrial RNA localisation, mtRNA localization